{
  "gene_symbol": "MUC7",
  "gene": "UniProtKB:Q8TAX7",
  "term_id": "UNKNOWN:0002",
  "gene_name": "Mucin-7",
  "term_label": "Unknown biological process"
}